memory T cell differentiation [GO:0043379] (BP) Sources: ISBN:0781735149 Also known as: memory T lymphocyte differentiation, memory T-cell differentiation, memory T-lymphocyte differentiation, memory T cell development Regulation: regulated by regulation of memory T cell differentiation [GO:0043380]; negatively regulated by negative regulation of memory T cell differentiation [GO:0043381]; positively regulated by positive regulation of memory T cell differentiation [GO:0043382] Note: Note that immunologists typically use the word 'development' to refer to cells of B or T cell lineages undergoing the process that GO describes as 'cell differentiation'. Definition: The process in which a newly activated T cell acquires specialized features of a memory T cell. Relationships: is a type of T cell differentiation involved in immune response [GO:0002292]; is a type of immunological memory formation process [GO:0090715]